mitochondrial membrane scission site [GO:0090692] (cellular component) Definition: The site on the mitochondrial membrane where the separation of a single continuous mitochondrial membrane into two membranes occurs as a final step in mitochondrial fission. Relationships: is_a cellular anatomical structure [GO:0110165]; is part of GO:0031966 References: PMID:26618722 Sources: GOC:PARL, GOC:bc